{
  "term_label": "Unknown cellular component",
  "gene_symbol": "NBPF20",
  "gene_name": "Neuroblastoma breakpoint family member 20",
  "term_id": "UNKNOWN:0003",
  "gene": "UniProtKB:P0DPF2"
}